multi-layer follicle stage [GO:0048162] (biological process) Definition: The stage in oogenesis when many layers of follicle cells surround the oocyte. There is a yolk nucleus (Balbiani's Body) near the germinal vesicle. Also known as: mammalian oogenesis stage 5 Relationships: is_a GO:0022605 Sources: GOC:jid, GOC:mtg_sensu, ISBN:0198542771